{
  "term_id": "GO:0008285",
  "gene": "UniProtKB:Q92574",
  "gene_name": "Hamartin",
  "gene_symbol": "TSC1",
  "term_label": "negative regulation of cell population proliferation"
}